{
  "gene_name": "High affinity choline transporter 1",
  "gene_symbol": "SLC5A7",
  "gene": "UniProtKB:Q9GZV3",
  "term_label": "plasma membrane",
  "term_id": "GO:0005886"
}